tyrosine metabolic process [GO:0006570] (biological process) Subtypes: GO:0006571, GO:0006572, melanin biosynthetic process from tyrosine [GO:0006583], GO:0006585 Also known as: tyrosine metabolism Relationships: is a type of aromatic amino acid metabolic process [GO:0009072]; is a type of GO:0170033; is a type of proteinogenic amino acid metabolic process [GO:0170039] Sources: GOC:go_curators Definition: The chemical reactions and pathways involving tyrosine, an aromatic amino acid, 2-amino-3-(4-hydroxyphenyl)propanoic acid.